{
  "gene_name": "Cyclin-D-binding Myb-like transcription factor 1",
  "gene_symbol": "DMTF1",
  "gene": "UniProtKB:Q9Y222",
  "term_id": "GO:0000978",
  "term_label": "RNA polymerase II cis-regulatory region sequence-specific DNA binding"
}